{
  "term_id": "GO:0006606",
  "gene_name": "Importin-7",
  "term_label": "protein import into nucleus",
  "gene_symbol": "IPO7",
  "gene": "UniProtKB:O95373"
}